intracellular mRNA localization involved in anterior/posterior axis specification [GO:0060811] (biological process) Definition: Any process in which mRNA is transported to, or maintained in, a specific location within the oocyte and/or syncytial embryo that contributes to the specification of the anterior/posterior axis. Sources: GOC:dph, GOC:sdb_2009, GOC:tb Subtypes: GO:0019094, bicoid mRNA localization [GO:0045450], orthodenticle mRNA localization [GO:0060812], anterior mRNA localization involved in anterior/posterior axis specification [GO:0060813], posterior mRNA localization involved in anterior/posterior axis specification [GO:0060814] Also known as: intracellular mRNA localisation involved in anterior/posterior axis specification Relationships: is a type of GO:0060810; is part of anterior/posterior axis specification [GO:0009948]